ketone metabolic process [GO:0042180] (biological process) Regulation: regulated by regulation of ketone metabolic process [GO:0010565] Relationships: is_a metabolic process [GO:0008152] Also known as: ketone metabolism Sources: GOC:jl, ISBN:0787650153 Definition: The chemical reactions and pathways involving any of a class of organic compounds that contain the carbonyl group, CO, and in which the carbonyl group is bonded only to carbon atoms, as carried out by individual cells. The general formula for a ketone is RCOR, where R and R are alkyl or aryl groups. Subtypes: 3-keto-sphinganine metabolic process [GO:0006666], menaquinone metabolic process [GO:0009233], methylglyoxal metabolic process [GO:0009438], citrate catabolic process to diacetyl [GO:0019651], 1-(3,5-dichloro-2,6-dihydroxy-4-methoxyphenyl)hexan-1-one metabolic process [GO:0031147], aldosterone metabolic process [GO:0032341], cortisol metabolic process [GO:0034650], asperthecin metabolic process [GO:0036182], ketone biosynthetic process [GO:0042181], ketone catabolic process [GO:0042182], vitamin K metabolic process [GO:0042373], progesterone metabolic process [GO:0042448], GO:0044597, doxorubicin metabolic process [GO:0044598], acetoin metabolic process [GO:0045149], ecdysteroid metabolic process [GO:0045455], glycerol to glycerone phosphate metabolic process [GO:0061610], GO:0061720, GO:0062173, kynurenine metabolic process [GO:0070189], monodictyphenone metabolic process [GO:1900813], quinone metabolic process [GO:1901661], (25S)-Delta(7)-dafachronate metabolic process [GO:1902056]